{
  "term_id": "GO:0005886",
  "gene": "UniProtKB:Q15619",
  "gene_name": "Olfactory receptor 1C1",
  "gene_symbol": "OR1C1",
  "term_label": "plasma membrane"
}